positive regulation of protein K63-linked deubiquitination [GO:1903006] (biological process) Definition: Any process that activates or increases the frequency, rate or extent of protein K63-linked deubiquitination. References: PMID:22970133 Sources: GOC:PARL, GOC:TermGenie, GOC:bf, GO_REF:0000058 Relationships: is a type of positive regulation of protein deubiquitination [GO:1903003]; is a type of regulation of protein K63-linked deubiquitination [GO:1903004]; positively regulates protein K63-linked deubiquitination [GO:0070536] Also known as: up regulation of protein K63-linked deubiquitination, up-regulation of protein K63-linked deubiquitination, upregulation of protein K63-linked deubiquitination, activation of protein K63-linked deubiquitination